positive regulation of arabinoxylan-containing compound catabolic process [GO:2000923] (biological process) Subtypes: positive regulation of glucuronoarabinoxylan catabolic process [GO:2000920] Sources: GOC:mengo_curators Also known as: positive regulation of arabinoxylan catabolism Definition: Any process that activates or increases the frequency, rate or extent of arabinoxylan-containing compound catabolic process. Relationships: is a type of regulation of arabinoxylan-containing compound catabolic process [GO:2000921]; is a type of GO:2001002; positively regulates arabinoxylan-containing compound catabolic process [GO:2000888]